{
  "gene": "UniProtKB:P02461",
  "term_id": "GO:0048705",
  "gene_name": "Collagen alpha-1(III) chain",
  "term_label": "skeletal system morphogenesis",
  "gene_symbol": "COL3A1"
}